microtubule nucleation by interphase microtubule organizing center [GO:0051415] (biological process) Definition: The 'de novo' formation of a microtubule by the interphase microtubule organizing center during interphase, the stage of cell cycle between successive rounds of chromosome segregation. Sources: GOC:ai Also known as: IMTOC-mediated microtubule nucleation during interphase, interphase microtubule nucleation by interphase microtubule organising centre, interphase microtubule nucleation by interphase microtubule organizing center, interphase microtubule organizing center-mediated microtubule nucleation during interphase, microtubule nucleation during interphase by IMTOC, microtubule nucleation during interphase by interphase microtubule organizing center Relationships: is a type of microtubule nucleation by microtubule organizing center [GO:0051418]